{
  "gene_name": "Eyes absent homolog 3",
  "term_label": "positive regulation of DNA repair",
  "gene_symbol": "EYA3",
  "term_id": "GO:0045739",
  "gene": "UniProtKB:Q99504"
}